{
  "gene_symbol": "SRGAP2",
  "gene": "UniProtKB:O75044",
  "term_label": "negative regulation of cell migration",
  "term_id": "GO:0030336",
  "gene_name": "SLIT-ROBO Rho GTPase-activating protein 2"
}